{
  "term_label": "extrinsic apoptotic signaling pathway",
  "gene_symbol": "TNFRSF1B",
  "gene_name": "Tumor necrosis factor receptor superfamily member 1B",
  "gene": "UniProtKB:P20333",
  "term_id": "GO:0097191"
}